{
  "term_id": "GO:0045275",
  "gene": "UniProtKB:P07919",
  "gene_symbol": "UQCRH",
  "term_label": "respiratory chain complex III",
  "gene_name": "Cytochrome b-c1 complex subunit 6, mitochondrial"
}